positive regulation of polyketide biosynthetic process [GO:1900734] (biological process) Definition: Any process that activates or increases the frequency, rate or extent of polyketide biosynthetic process. Sources: GOC:TermGenie, GOC:di Also known as: activation of polyketide anabolism, activation of polyketide biosynthesis, activation of polyketide formation, activation of polyketide synthesis, positive regulation of polyketide anabolism, positive regulation of polyketide biosynthesis, positive regulation of polyketide formation, positive regulation of polyketide synthesis, up regulation of polyketide anabolism, up regulation of polyketide biosynthesis, up regulation of polyketide biosynthetic process, up regulation of polyketide formation, up regulation of polyketide synthesis, up-regulation of polyketide anabolism, up-regulation of polyketide biosynthesis, up-regulation of polyketide biosynthetic process, up-regulation of polyketide formation, up-regulation of polyketide synthesis, upregulation of polyketide anabolism, upregulation of polyketide biosynthesis, upregulation of polyketide biosynthetic process, upregulation of polyketide formation, upregulation of polyketide synthesis, activation of polyketide biosynthetic process Subtypes: positive regulation of patulin biosynthetic process [GO:0140724], GO:0140736, GO:1900639, positive regulation of F-9775A biosynthetic process [GO:1900672], positive regulation of F-9775B biosynthetic process [GO:1900677], positive regulation of neosartoricin biosynthetic process [GO:1902055] Relationships: is a type of positive regulation of secondary metabolite biosynthetic process [GO:1900378]; is a type of regulation of polyketide biosynthetic process [GO:1900732]; positively regulates polyketide biosynthetic process [GO:0030639]